maltose transmembrane transporter activity [GO:0005363] (molecular function) Sources: GOC:mtg_transport, ISBN:0198506732, ISBN:0815340729 Also known as: maltose porter activity Definition: Enables the transfer of maltose from one side of a membrane to the other. Maltose is the disaccharide 4-O-alpha-D-glucopyranosyl-D-glucopyranose, an intermediate in the enzymatic breakdown of glycogen and starch. Subtypes: GO:0005364, ABC-type maltose transporter activity [GO:0015423], maltose transporting porin activity [GO:0015481], GO:0022873 Relationships: is a type of GO:0015154; is part of maltose transport [GO:0015768]